regulation of [2Fe-2S] cluster assembly [GO:1900487] (biological process) Relationships: is a type of regulation of iron-sulfur cluster assembly [GO:1903329]; regulates [2Fe-2S] cluster assembly [GO:0044571] Definition: Any process that modulates the frequency, rate or extent of [2Fe-2S] cluster assembly. Subtypes: negative regulation of [2Fe-2S] cluster assembly [GO:1900488], positive regulation of [2Fe-2S] cluster assembly [GO:1900489] Also known as: regulation of 2Fe-2S cluster assembly, regulation of [2Fe-2S] cluster biosynthetic process Sources: GOC:TermGenie, GOC:mengo_curators, GOC:pr